{
  "term_id": "GO:0030838",
  "term_label": "positive regulation of actin filament polymerization",
  "gene_name": "Cdc42 effector protein 4",
  "gene_symbol": "CDC42EP4",
  "gene": "UniProtKB:Q9H3Q1"
}